{
  "gene": "UniProtKB:Q93099",
  "term_label": "L-phenylalanine catabolic process",
  "gene_symbol": "HGD",
  "gene_name": "Homogentisate 1,2-dioxygenase",
  "term_id": "GO:0006559"
}